{
  "gene_name": "Histone H2B type F-S",
  "term_id": "GO:0006325",
  "term_label": "chromatin organization",
  "gene": "UniProtKB:P57053",
  "gene_symbol": "H2BC12L"
}